{
  "gene_name": "Synaptosomal-associated protein 29",
  "term_id": "GO:0006887",
  "gene_symbol": "SNAP29",
  "term_label": "exocytosis",
  "gene": "UniProtKB:O95721"
}